{
  "gene_symbol": "PTPN21",
  "gene_name": "Tyrosine-protein phosphatase non-receptor type 21",
  "gene": "UniProtKB:Q16825",
  "term_label": "positive regulation of hippo signaling",
  "term_id": "GO:0035332"
}